{
  "gene_symbol": "GAD2",
  "term_id": "GO:0006540",
  "term_label": "gamma-aminobutyrate shunt",
  "gene": "UniProtKB:Q05329",
  "gene_name": "Glutamate decarboxylase 2"
}